lysine catabolic process [GO:0006554] (biological process) Definition: The chemical reactions and pathways resulting in the breakdown of lysine, 2,6-diaminohexanoic acid. Also known as: lysine breakdown, lysine catabolism, lysine degradation Sources: GOC:go_curators Relationships: is a type of GO:0006553; is a type of GO:1901606 Subtypes: D-lysine catabolic process [GO:0019476], GO:0019477